{
  "term_label": "galanin receptor activity",
  "gene_name": "Cysteinyl leukotriene receptor 1",
  "term_id": "GO:0004966",
  "gene_symbol": "CYSLTR1",
  "gene": "UniProtKB:Q9Y271"
}